positive regulation of gene expression, epigenetic [GO:0141137] (biological process) Subtypes: transcription initiation-coupled chromatin remodeling [GO:0045815], chromosomal 5-methylcytosine DNA demethylation, oxidation pathway [GO:0141167] Relationships: is a type of positive regulation of gene expression [GO:0010628]; is a type of epigenetic regulation of gene expression [GO:0040029] References: PMID:36618446 Definition: An epigenetic process that increases gene expression at specific genomic regions through chromatin remodeling either by modifying higher order chromatin fiber structure, nucleosomal histones, or the cytosine DNA demethylation. Also known as: activation of gene expression, epigenetic, up regulation of gene expression, epigenetic, up-regulation of gene expression, epigenetic, upregulation of gene expression, epigenetic